{
  "term_id": "GO:0005829",
  "term_label": "cytosol",
  "gene_symbol": "PABPC1",
  "gene_name": "Polyadenylate-binding protein 1",
  "gene": "UniProtKB:P11940"
}